{
  "gene": "UniProtKB:Q14721",
  "term_label": "postsynaptic membrane",
  "gene_name": "Potassium voltage-gated channel subfamily B member 1",
  "gene_symbol": "KCNB1",
  "term_id": "GO:0045211"
}